{
  "term_id": "GO:0005829",
  "gene_symbol": "AKR1C4",
  "gene": "UniProtKB:P17516",
  "gene_name": "Aldo-keto reductase family 1 member C4",
  "term_label": "cytosol"
}